{
  "gene": "UniProtKB:Q8WWY8",
  "gene_symbol": "LIPH",
  "term_id": "GO:0004620",
  "gene_name": "Lipase member H",
  "term_label": "phospholipase activity"
}